regulation of animal organ morphogenesis [GO:2000027] (BP) Also known as: regulation of histogenesis and organogenesis Subtypes: regulation of animal organ formation [GO:0003156], regulation of polarized epithelial cell differentiation [GO:0030860], regulation of odontogenesis [GO:0042481], regulation of mesodermal cell fate specification [GO:0042661], GO:0048334, GO:0060651, regulation of branching involved in salivary gland morphogenesis [GO:0060693], regulation of branching involved in mammary gland duct morphogenesis [GO:0060762], positive regulation of posterior neural plate formation by fibroblast growth factor receptor signaling pathway [GO:0060787], GO:0072106, regulation of establishment of planar polarity [GO:0090175], regulation of branching involved in ureteric bud morphogenesis [GO:0090189], GO:0110041, positive regulation of animal organ morphogenesis [GO:0110110], GO:0110111, regulation of chondrocyte differentiation involved in endochondral bone morphogenesis [GO:1902738], regulation of otic vesicle morphogenesis [GO:1904118], regulation of metanephric S-shaped body morphogenesis [GO:2000004], regulation of metanephric comma-shaped body morphogenesis [GO:2000006], regulation of heart morphogenesis [GO:2000826] Definition: Any process that modulates the frequency, rate or extent of animal organ morphogenesis. Sources: GOC:obol Relationships: is a type of regulation of anatomical structure morphogenesis [GO:0022603]; regulates animal organ morphogenesis [GO:0009887]